{
  "gene_name": "Ubiquitin-like modifier-activating enzyme 5",
  "gene": "UniProtKB:Q9GZZ9",
  "term_label": "protein ufmylation",
  "term_id": "GO:0071569",
  "gene_symbol": "UBA5"
}